{
  "gene": "UniProtKB:O60469",
  "gene_symbol": "DSCAM",
  "gene_name": "Cell adhesion molecule DSCAM",
  "term_label": "plasma membrane",
  "term_id": "GO:0005886"
}